{
  "gene": "UniProtKB:P35575",
  "gene_name": "Glucose-6-phosphatase catalytic subunit 1",
  "term_id": "GO:0004346",
  "term_label": "glucose-6-phosphatase activity",
  "gene_symbol": "G6PC1"
}